{
  "term_id": "UNKNOWN:0003",
  "gene_name": "Serine-rich coiled-coil domain-containing protein 1",
  "term_label": "Unknown cellular component",
  "gene_symbol": "CCSER1",
  "gene": "UniProtKB:Q9C0I3"
}